{
  "gene": "UniProtKB:Q86VP6",
  "gene_symbol": "CAND1",
  "term_label": "protein ubiquitination",
  "term_id": "GO:0016567",
  "gene_name": "Cullin-associated NEDD8-dissociated protein 1"
}